negative regulation of protein localization to non-growing cell tip [GO:0062108] (biological process) References: PMID:18328707 Relationships: is a type of GO:0062107; is a type of negative regulation of protein localization to cell tip [GO:1903067]; negatively regulates protein localization to non-growing cell tip [GO:1902487] Definition: Any process that stops, prevents or reduces the frequency, rate or extent of protein localization to a non-growing cell tip.